{
  "gene": "UniProtKB:Q17RM4",
  "gene_name": "Coiled-coil domain-containing protein 142",
  "gene_symbol": "CCDC142",
  "term_label": "Unknown molecular function",
  "term_id": "UNKNOWN:0001"
}